{
  "gene_symbol": "TRDN",
  "gene_name": "Triadin",
  "term_label": "protein-macromolecule adaptor activity",
  "term_id": "GO:0030674",
  "gene": "UniProtKB:Q13061"
}